{
  "term_label": "Unknown molecular function",
  "term_id": "UNKNOWN:0001",
  "gene": "UniProtKB:A0A075B6I6",
  "gene_symbol": "IGLV1-50",
  "gene_name": "Probable non-functional immunoglobulin lambda variable 1-50"
}